spliceosomal snRNP assembly [GO:0000387] (BP) Definition: The aggregation, arrangement and bonding together of one or more snRNA and multiple protein components to form a ribonucleoprotein complex that is involved in formation of the spliceosome. Sources: GOC:krc, GOC:mah, ISBN:0879695897 Also known as: spliceosomal snRNP biogenesis Relationships: is a type of protein-RNA complex assembly [GO:0022618]; is part of mRNA splicing, via spliceosome [GO:0000398] Subtypes: spliceosomal tri-snRNP complex assembly [GO:0000244]